{
  "term_label": "Unknown molecular function",
  "term_id": "UNKNOWN:0001",
  "gene": "UniProtKB:A0A1B0GXF2",
  "gene_symbol": "TRBV7-2",
  "gene_name": "T cell receptor beta variable 7-2"
}